{
  "gene_symbol": "ZNF710",
  "term_id": "GO:0006357",
  "gene": "UniProtKB:Q8N1W2",
  "term_label": "regulation of transcription by RNA polymerase II",
  "gene_name": "Zinc finger protein 710"
}